{
  "gene_name": "Large ribosomal subunit protein mL41",
  "term_id": "GO:0006412",
  "gene_symbol": "MRPL41",
  "gene": "UniProtKB:Q8IXM3",
  "term_label": "translation"
}